16S rRNA (guanine(1516)-N(2))-methyltransferase activity [GO:0036308] (molecular function) References: PMID:22079366 Sources: GOC:imk Relationships: is_a rRNA (guanine-N2-)-methyltransferase activity [GO:0008990] Definition: Catalysis of the reaction: S-adenosyl-L-methionine + guanosine(1516) in 16S rRNA = N(2)-methylguanosine(1516) in 16S rRNA + S-adenosyl-L-homocysteine.